{
  "term_id": "GO:0043022",
  "gene": "UniProtKB:Q9BY44",
  "gene_symbol": "EIF2A",
  "gene_name": "Eukaryotic translation initiation factor 2A",
  "term_label": "ribosome binding"
}